{
  "term_label": "protein kinase CK2 complex",
  "gene_name": "Casein kinase II subunit alpha 3",
  "gene": "UniProtKB:Q8NEV1",
  "term_id": "GO:0005956",
  "gene_symbol": "CSNK2A3"
}